{
  "gene_symbol": "TMEM86B",
  "term_label": "Unknown biological process",
  "gene_name": "Lysoplasmalogenase",
  "gene": "UniProtKB:Q8N661",
  "term_id": "UNKNOWN:0002"
}